{
  "term_id": "GO:1902531",
  "term_label": "regulation of intracellular signal transduction",
  "gene_symbol": "ANKRD54",
  "gene_name": "Ankyrin repeat domain-containing protein 54",
  "gene": "UniProtKB:Q6NXT1"
}